positive regulation of type II hypersensitivity [GO:0002894] (biological process) Sources: GOC:add Subtypes: positive regulation of type IIa hypersensitivity [GO:0001798], positive regulation of type IIb hypersensitivity [GO:0001801] Definition: Any process that activates or increases the frequency, rate, or extent of type II hypersensitivity. Also known as: up regulation of type II hypersensitivity, up-regulation of type II hypersensitivity, upregulation of type II hypersensitivity, activation of type II hypersensitivity, stimulation of type II hypersensitivity Relationships: is a type of positive regulation of hypersensitivity [GO:0002885]; is a type of positive regulation of myeloid leukocyte mediated immunity [GO:0002888]; is a type of GO:0002891; is a type of regulation of type II hypersensitivity [GO:0002892]; positively regulates type II hypersensitivity [GO:0002445]